{
  "gene_symbol": "TMED4",
  "term_id": "GO:0006888",
  "gene_name": "Transmembrane emp24 domain-containing protein 4",
  "gene": "UniProtKB:Q7Z7H5",
  "term_label": "endoplasmic reticulum to Golgi vesicle-mediated transport"
}